hydrogen metabolic process [GO:1902421] (biological process) Definition: The chemical reactions and pathways involving H2 (dihydrogen). Relationships: is a type of metabolic process [GO:0008152] References: PMID:20395274, PMID:20692761 Sources: GOC:TermGenie, GOC:mengo_curators Subtypes: hydrogen biosynthetic process [GO:1902422], methane biosynthetic process from methanol and hydrogen [GO:1990491] Also known as: H2 metabolism, dihydrogen metabolism, molecular hydrogen metabolism